{
  "term_label": "apical junction complex",
  "gene_symbol": "NECTIN3",
  "gene": "UniProtKB:Q9NQS3",
  "term_id": "GO:0043296",
  "gene_name": "Nectin-3"
}